interleukin-9 production [GO:0032638] (biological process) Sources: GOC:mah Relationships: is a type of cytokine production [GO:0001816] Definition: The appearance of interleukin-9 due to biosynthesis or secretion following a cellular stimulus, resulting in an increase in its intracellular or extracellular levels. Also known as: IL-9 production, interleukin-9 biosynthetic process, interleukin-9 secretion Regulation: regulated by regulation of interleukin-9 production [GO:0032678]; negatively regulated by negative regulation of interleukin-9 production [GO:0032718]; positively regulated by positive regulation of interleukin-9 production [GO:0032758]